cellulose-polysulfatase activity [GO:0033886] (molecular function) Also known as: cellulose-sulfate sulfohydrolase activity Relationships: is a type of GO:0008484 Definition: Catalysis of the hydrolysis of the 2- and 3-sulfate groups of the polysulfates of cellulose and charonin. Sources: EC:3.1.6.7